{
  "gene": "UniProtKB:A6NFC9",
  "gene_symbol": "OR2W5P",
  "term_label": "plasma membrane",
  "gene_name": "Putative olfactory receptor 2W5 pseudogene",
  "term_id": "GO:0005886"
}